{
  "gene_symbol": "TRMT61A",
  "gene": "UniProtKB:Q96FX7",
  "term_label": "tRNA methylation",
  "term_id": "GO:0030488",
  "gene_name": "tRNA (adenine(58)-N(1))-methyltransferase catalytic subunit TRMT61A"
}